{
  "term_label": "regulation of stress fiber assembly",
  "gene_name": "Arf-GAP with SH3 domain, ANK repeat and PH domain-containing protein 3",
  "gene": "UniProtKB:Q8TDY4",
  "gene_symbol": "ASAP3",
  "term_id": "GO:0051492"
}